{
  "term_id": "GO:0004222",
  "gene_name": "Matrix metalloproteinase-26",
  "term_label": "metalloendopeptidase activity",
  "gene_symbol": "MMP26",
  "gene": "UniProtKB:Q9NRE1"
}